{
  "gene_symbol": "KLHL41",
  "term_id": "GO:2001014",
  "gene": "UniProtKB:O60662",
  "term_label": "regulation of skeletal muscle cell differentiation",
  "gene_name": "Kelch-like protein 41"
}